{
  "gene": "UniProtKB:O95727",
  "term_id": "GO:0005102",
  "gene_name": "Cytotoxic and regulatory T-cell molecule",
  "term_label": "signaling receptor binding",
  "gene_symbol": "CRTAM"
}